negative regulation of corticosterone secretion [GO:2000853] (biological process) Definition: Any process that stops, prevents or reduces the frequency, rate or extent of corticosterone secretion. Sources: GOC:sl Relationships: is a type of negative regulation of glucocorticoid secretion [GO:2000850]; is a type of regulation of corticosterone secretion [GO:2000852]; negatively regulates corticosterone secretion [GO:0035934]